cellular response to amino acid starvation [GO:0034198] (biological process) Also known as: GAAC response, general amino acid control response Sources: GOC:ecd Subtypes: cellular response to leucine starvation [GO:1990253] Definition: Any process that results in a change in state or activity of a cell (in terms of movement, secretion, enzyme production, gene expression, etc.) as a result of deprivation of amino acids. Relationships: is_a cellular response to starvation [GO:0009267]; is a type of response to amino acid starvation [GO:1990928] Regulation: negatively regulated by negative regulation of cellular response to amino acid starvation [GO:1903574]; regulated by regulation of cellular response to amino acid starvation [GO:1903832]; positively regulated by positive regulation of cellular response to amino acid starvation [GO:1903833]